3-galactosyl-N-acetylglucosaminide 4-alpha-L-fucosyltransferase activity [GO:0017060] (molecular function) Sources: EC:2.4.1.65 Also known as: (Le(a))-dependent (alpha-3/4)-fucosyltransferase activity, (Lea)-dependent (alpha-3/4)-fucosyltransferase activity, FucT-II activity, Lewis FT activity, Lewis alpha-(1,3/4)-fucosyltransferase activity, Lewis alpha-(1->3/4)-fucosyltransferase activity, Lewis blood group alpha-(1,3/4)-fucosyltransferase activity, Lewis blood group alpha-(1->3/4)-fucosyltransferase activity, Lewis(Le) blood group gene-dependent alpha-(1,3/4)-L-fucosyltransferase activity, alpha(1,4)-L-fucosyltransferase activity, alpha-(1,3/1,4) fucosyltransferase III activity, alpha-(1,4)-L-fucosyltransferase activity, alpha-(1->4)-L-fucosyltransferase activity, alpha-4-L-fucosyltransferase activity, beta-acetylglucosaminylsaccharide fucosyltransferase activity, blood group Lewis alpha-4-fucosyltransferase activity, blood-group substance Le(a)-dependent fucosyltransferase activity, blood-group substance Lea-dependent fucosyltransferase, galactoside 3(4)-L-fucosyltransferase activity, Lewis(Le) blood group gene-dependent alpha-(1->3/4)-L-fucosyltransferase activity, 3-alpha-galactosyl-N-acetylglucosaminide 4-alpha-L-fucosyltransferase activity, GDP-L-fucose:3-beta-D-galactosyl-N-acetyl-D-glucosaminyl-R 4I-alpha-L-fucosyltransferase activity, GDP-beta-L-fucose:3-beta-D-galactosyl-N-acetyl-D-glucosaminyl-R 4I-alpha-L-fucosyltransferase activity, fuca(1,3)-glycosidic linkage formation, guanosine diphosphofucose-beta-acetylglucosaminylsaccharide 4-alpha-L-fucosyltransferase activity, guanosine diphosphofucose-glycoprotein 4-alpha-L-fucosyltransferase activity, guanosine diphosphofucose-glycoprotein 4-alpha-fucosyltransferase activity Relationships: is a type of fucosyltransferase activity [GO:0008417] Definition: Catalysis of the reaction: GDP-L-fucose + beta-D-galactosyl-(1,3)-N-acetyl-D-glucosaminyl-R = GDP + beta-D-galactosyl-(1,3)-[alpha-L-fucosyl-(1,4)]-N-acetyl-D-glucosaminyl-R.